o-aminophenol oxidase activity [GO:0050149] (molecular function) Relationships: is_a oxidoreductase activity, acting on diphenols and related substances as donors, oxygen as acceptor [GO:0016682] Sources: EC:1.10.3.4, MetaCyc:O-AMINOPHENOL-OXIDASE-RXN Also known as: 2-aminophenol:O2 oxidoreductase activity, 2-aminophenol:oxygen oxidoreductase activity, GriF, isophenoxazine synthase activity, o-aminophenol:O2 oxidoreductase activity Definition: Catalysis of the reaction: 2 2-aminophenol + 3 O2 = 2 isophenoxazine + 6 H2O.